{
  "gene": "UniProtKB:P08217",
  "gene_symbol": "CELA2A",
  "term_label": "extracellular space",
  "term_id": "GO:0005615",
  "gene_name": "Chymotrypsin-like elastase family member 2A"
}